cuticle development involved in collagen and cuticulin-based cuticle molting cycle [GO:0042338] (biological process) Relationships: is_a collagen and cuticulin-based cuticle development [GO:0040002]; is part of molting cycle, collagen and cuticulin-based cuticle [GO:0018996] Sources: GOC:mtg_sensu Also known as: cuticle anabolism during molting, cuticle biosynthetic process during molting, cuticle formation during molting, cuticle synthesis during molting, collagen and cuticulin-based cuticle development during molting Definition: Synthesis and deposition of a collagen and cuticulin-based noncellular, hardened, or membranous secretion from an epithelial sheet, occurring as part of the molting cycle. An example of this process is found in Caenorhabditis elegans.